sexual spore wall assembly [GO:0034294] (biological process) Also known as: sexual spore wall formation Relationships: is a type of GO:0003006; is a type of spore wall assembly [GO:0042244]; is_a GO:1903046; is part of sexual sporulation [GO:0034293] Sources: GOC:mah Definition: The aggregation, arrangement and bonding together of a set of components to form a sexual spore wall, the specialized envelope lying outside the cell membrane of a spore derived from a product of meiosis.